cell killing [GO:0001906] (biological process) Definition: Any process in an organism that results in the killing of its own cells or those of another organism, including in some cases the death of the other organism. Killing here refers to the induction of death in one cell by another cell, not cell-autonomous death due to internal or other environmental conditions. Sources: GOC:add Also known as: necrosis Relationships: is a type of cellular process [GO:0009987] Subtypes: GO:0001909, killing of cells of another organism [GO:0031640], complement-dependent cytotoxicity [GO:0097278] Regulation: regulated by regulation of cell killing [GO:0031341]; negatively regulated by negative regulation of cell killing [GO:0031342]; positively regulated by positive regulation of cell killing [GO:0031343]